{
  "term_label": "Unknown cellular component",
  "gene_name": "Uncharacterized protein",
  "gene_symbol": "A0A0G2JLW4",
  "term_id": "UNKNOWN:0003",
  "gene": "UniProtKB:A0A0G2JLW4"
}